{
  "term_label": "peroxisome fission",
  "term_id": "GO:0016559",
  "gene_symbol": "FIS1",
  "gene": "UniProtKB:Q9Y3D6",
  "gene_name": "Mitochondrial fission 1 protein"
}